{
  "gene": "UniProtKB:Q9BXJ2",
  "term_label": "Unknown cellular component",
  "gene_symbol": "C1QTNF7",
  "term_id": "UNKNOWN:0003",
  "gene_name": "Complement C1q tumor necrosis factor-related protein 7"
}